phosphatidylserine-phosphatidylinositol-4-phosphate exchange activity [GO:0160270] (molecular function) References: PMID:34249917, PMID:39106189 Sources: RHEA:81667 Definition: Catalysis of the reaction: a 1,2-diacyl-sn-glycero-3-phospho-(1D-myo-inositol 4-phosphate)(out) + a 1,2-diacyl-sn-glycero-3-phospho-L-serine(in) = a 1,2-diacyl-sn-glycero-3-phospho-(1D-myo-inositol 4-phosphate)(in) + a 1,2-diacyl-sn-glycero-3-phospho-L-serine(out). This reaction results in the exchange of phosphatidylserine (PS) for phosphatidylinositol-4-phosphate (PI(4)P) between membranes. Relationships: is a type of phosphatidylinositol transfer activity [GO:0008526]; is a type of GO:0140343; is a type of lipid exchange activity [GO:7770011]